{
  "gene": "UniProtKB:Q9UKT6",
  "term_id": "GO:0043153",
  "gene_name": "Putative F-box_LRR-repeat protein 21",
  "gene_symbol": "FBXL21P",
  "term_label": "entrainment of circadian clock by photoperiod"
}